dTDP biosynthetic process [GO:0006233] (biological process) Also known as: dTDP anabolism, dTDP biosynthesis, dTDP formation, dTDP synthesis Definition: The chemical reactions and pathways resulting in the formation of dTDP, deoxyribosylthymine diphosphate (2'-deoxyribosylthymine5'-diphosphate). Relationships: is_a pyrimidine deoxyribonucleoside diphosphate biosynthetic process [GO:0009197]; is a type of pyrimidine deoxyribonucleotide biosynthetic process [GO:0009221]; is a type of dTDP metabolic process [GO:0046072] Sources: ISBN:0198506732